{
  "gene_symbol": "RPP21",
  "gene": "UniProtKB:Q9H633",
  "term_id": "GO:0005655",
  "gene_name": "Ribonuclease P protein subunit p21",
  "term_label": "nucleolar ribonuclease P complex"
}